{
  "gene_symbol": "SHMT1",
  "gene": "UniProtKB:P34896",
  "term_id": "GO:0030170",
  "term_label": "pyridoxal phosphate binding",
  "gene_name": "Serine hydroxymethyltransferase, cytosolic"
}